galactosylceramidase activity [GO:0004336] (molecular function) Definition: Catalysis of the reaction: D-galactosyl-N-acylsphingosine + H2O = D-galactose + N-acylsphingosine. Sources: EC:3.2.1.46 Also known as: D-galactosyl-N-acylsphingosine galactohydrolase activity, beta-galactocerebrosidase activity, beta-galactosylceramidase activity, ceramide galactosidase activity, cerebroside beta-galactosidase activity, cerebroside galactosidase activity, galactocerebrosidase activity, galactocerebroside beta-galactosidase activity, galactocerebroside galactosidase activity, galactocerebroside-beta-D-galactosidase activity, galactosylceramidase I, galactosylceramide beta-galactosidase activity, galactosylcerebrosidase activity, galcerase activity, lactosylceramidase I, lactosylceramidase activity Relationships: is a type of glycosylceramidase activity [GO:0017042]